{
  "gene_name": "Sodium_potassium-transporting ATPase subunit beta-3",
  "gene": "UniProtKB:P54709",
  "gene_symbol": "ATP1B3",
  "term_id": "GO:0030007",
  "term_label": "intracellular potassium ion homeostasis"
}